{
  "term_id": "GO:0007169",
  "gene_symbol": "EPHA2",
  "gene": "UniProtKB:P29317",
  "gene_name": "Ephrin type-A receptor 2",
  "term_label": "cell surface receptor protein tyrosine kinase signaling pathway"
}